mesonephric extraglomerular mesangial cell proliferation involved in mesonephros development [GO:0061225] (biological process) Also known as: mesonephric Goormaghtigh proliferation, mesonephric lacis cell proliferation Relationships: is a type of cell proliferation involved in mesonephros development [GO:0061209]; is a type of extraglomerular mesangial cell proliferation [GO:0072122]; is part of GO:0061215 Definition: The multiplication or reproduction of extraglomerular glomerular mesangium cells in the mesonephros by cell division, resulting in the expansion of their population. Extraglomerular mesangial cells (also known as lacis cells, Goormaghtigh cells) are light-staining cells in the kidney found outside the glomerulus, near the vascular pole and macula densa. Sources: GOC:mtg_kidney_jan10